CFTR-NHERF-ezrin complex [GO:0034662] (cellular component) References: PMID:16129695, PMID:16798722, PMID:16926444 Relationships: is a type of plasma membrane protein complex [GO:0098797] Definition: A protein complex that contains ezrin, Na+/H+ exchanger regulatory factor (NHERF, also called EBP50), and two copies of the cystic fibrosis transmembrane conductance regulator (CFTR). The CFTR molecules interact with NHERF via their cytoplasmic tail domains; the complex is thought to link the CFTR channel to the actin cytoskeleton and contribute to the regulation of channel activity.